{
  "gene_name": "DNA mismatch repair protein Msh3",
  "term_label": "nucleus",
  "gene_symbol": "MSH3",
  "gene": "UniProtKB:P20585",
  "term_id": "GO:0005634"
}